positive regulation of ribosomal protein gene transcription by RNA polymerase II [GO:0060963] (BP) Definition: Any process that increases the frequency, rate or extent of the synthesis of RNA from ribosomal protein genes mediated by RNA polymerase II. Also known as: positive regulation of ribosomal protein gene transcription from RNA polymerase II promoter Sources: GOC:dph, GOC:tb, GOC:txnOH Relationships: is a type of positive regulation of transcription by RNA polymerase II [GO:0045944]; is a type of regulation of ribosomal protein gene transcription by RNA polymerase II [GO:0060962]